{
  "gene_name": "Unconventional myosin-Ia",
  "term_label": "endocytosis",
  "gene_symbol": "MYO1A",
  "term_id": "GO:0006897",
  "gene": "UniProtKB:Q9UBC5"
}